{
  "term_label": "Unknown biological process",
  "gene_name": "Ankyrin repeat and SOCS box protein 3",
  "gene_symbol": "ASB3",
  "gene": "UniProtKB:Q9Y575",
  "term_id": "UNKNOWN:0002"
}